{
  "term_label": "GDP-L-fucose synthase activity",
  "gene": "UniProtKB:Q13630",
  "term_id": "GO:0050577",
  "gene_name": "GDP-L-fucose synthase",
  "gene_symbol": "GFUS"
}